ocellus pigment metabolic process [GO:0046158] (biological process) Also known as: ocellus pigment metabolism References: PMID:15176085, PMID:18421706 Sources: GOC:ai Subtypes: ocellus pigment biosynthetic process [GO:0008055], ommochrome metabolic process [GO:0046152], GO:0046159 Relationships: is a type of secondary metabolic process [GO:0019748]; is_a pigment metabolic process involved in pigmentation [GO:0043474]; is part of ocellus pigmentation [GO:0033060] Definition: The chemical reactions and pathways involving ocellus pigments, any general or particular coloring matter in living organisms, found or utilized in the ocellus, a minute simple eye found in many invertebrates.